positive regulation of synaptic transmission, glutamatergic [GO:0051968] (biological process) Relationships: is a type of positive regulation of synaptic transmission [GO:0050806]; is_a regulation of synaptic transmission, glutamatergic [GO:0051966]; positively regulates GO:0035249 Also known as: up regulation of synaptic transmission, glutamatergic, up-regulation of synaptic transmission, glutamatergic, upregulation of synaptic transmission, glutamatergic, activation of synaptic transmission, glutamatergic, stimulation of synaptic transmission, glutamatergic Definition: Any process that activates, maintains or increases the frequency, rate or extent of glutamatergic synaptic transmission, the process of communication from a neuron to another neuron across a synapse using the neurotransmitter glutamate. Subtypes: positive regulation of glutamate secretion, neurotransmission [GO:1903296] Sources: GOC:ai